lysosome localization [GO:0032418] (biological process) Relationships: is a type of vacuolar localization [GO:1990849] Sources: GOC:mah Also known as: lysosome localisation Definition: Any process in which a lysosome is transported to, and/or maintained in, a specific location. Subtypes: mast cell degranulation [GO:0043303]